{
  "gene": "UniProtKB:Q13421",
  "term_id": "GO:0007160",
  "gene_symbol": "MSLN",
  "term_label": "cell-matrix adhesion",
  "gene_name": "Mesothelin"
}